{
  "term_id": "GO:0010508",
  "gene_symbol": "PLEKHF1",
  "gene_name": "Pleckstrin homology domain-containing family F member 1",
  "term_label": "positive regulation of autophagy",
  "gene": "UniProtKB:Q96S99"
}